{
  "term_id": "UNKNOWN:0001",
  "gene_symbol": "CENPV",
  "gene_name": "Centromere protein V",
  "term_label": "Unknown molecular function",
  "gene": "UniProtKB:Q7Z7K6"
}